intracellular sphingolipid homeostasis [GO:0090156] (biological process) Definition: A homeostatic process involved in the maintenance of a steady state level of sphingolipids within a cell. Also known as: cellular sphingolipid homeostasis Relationships: is a type of GO:0055082; is a type of lipid homeostasis [GO:0055088] Sources: GOC:ascb_2009, GOC:dph, GOC:tb